{
  "term_id": "GO:0032039",
  "gene_symbol": "INTS6L",
  "gene": "UniProtKB:Q5JSJ4",
  "gene_name": "Integrator complex subunit 6-like",
  "term_label": "integrator complex"
}